{
  "gene_name": "Lens fiber major intrinsic protein",
  "term_label": "apical plasma membrane",
  "term_id": "GO:0016324",
  "gene_symbol": "MIP",
  "gene": "UniProtKB:P30301"
}